RNA 2',3'-cyclic phosphatase activity [GO:0160272] (molecular function) Definition: Catalysis of the reaction: a 3'-end 2',3'-cyclophospho-ribonucleotide-RNA + 2 H2O = a 3'-end ribonucleotide-RNA + phosphate + H+. References: PMID:32732418 Relationships: is a type of phosphatase activity [GO:0016791]; is a type of catalytic activity, acting on RNA [GO:0140098]